chlorophyll metabolic process [GO:0015994] (biological process) Relationships: is a type of porphyrin-containing compound metabolic process [GO:0006778] Regulation: regulated by regulation of chlorophyll metabolic process [GO:0090056] Definition: The chemical reactions and pathways involving chlorophyll, any compound of magnesium complexed in a porphyrin (tetrapyrrole) ring and which functions as a photosynthetic pigment. Also known as: chlorophyll metabolism Subtypes: chlorophyll biosynthetic process [GO:0015995], chlorophyll catabolic process [GO:0015996], chlorophyll cycle [GO:0033354] Sources: GOC:jl